{
  "term_label": "nucleus",
  "term_id": "GO:0005634",
  "gene_name": "SMC5-SMC6 complex localization factor protein 2",
  "gene": "UniProtKB:Q8IX21",
  "gene_symbol": "SLF2"
}